glyphosate metabolic process [GO:0018920] (biological process) Definition: The chemical reactions and pathways involving glyphosate, a broad-spectrum herbicide also known by the trade name Roundup. It is a member of a broad class of compounds known as phosphonic acids, which contain a direct carbon-to-phosphorus (C-P) bond. Sources: UM-BBD_pathwayID:gly Also known as: Roundup metabolic process, Roundup metabolism, glyphosate metabolism Relationships: is a type of GO:0006575; is a type of phosphorus metabolic process [GO:0006793]; is a type of oxoacid metabolic process [GO:0043436]